vascular associated smooth muscle cell dedifferentiation [GO:1990936] (biological process) Relationships: is a type of GO:0090678 Also known as: vascular smooth muscle cell dedifferentiation Definition: The process in which a vascular smooth muscle cell (a non-striated, elongated, spindle-shaped cell found lining the blood vessels) loses the structural or functional features that characterize it in the mature organism, or some other relatively stable phase of the organism's life history. Under certain conditions, these cells can revert back to the features of the stem cells that were their ancestors. Regulation: regulated by regulation of vascular associated smooth muscle cell dedifferentiation [GO:1905174]; negatively regulated by negative regulation of vascular associated smooth muscle cell dedifferentiation [GO:1905175]; positively regulated by positive regulation of vascular associated smooth muscle cell dedifferentiation [GO:1905176] References: PMID:19088079 Sources: GOC:BHF, GOC:BHF_miRNA, GOC:rph